{
  "term_id": "UNKNOWN:0002",
  "gene_name": "Oxysterol-binding protein-related protein 9",
  "term_label": "Unknown biological process",
  "gene_symbol": "OSBPL9",
  "gene": "UniProtKB:Q96SU4"
}